mixed acid fermentation [GO:0019664] (biological process) Also known as: glucose catabolic process to mixed acids, glucose fermentation to mixed acids Definition: The anaerobic chemical reactions and pathways resulting in the breakdown of phosphoenolpyruvate into ethanol, lactate, formate, succinate, and acetate. Relationships: is_a ethanol metabolic process [GO:0006067]; is_a acetate metabolic process [GO:0006083]; is a type of lactate metabolic process [GO:0006089]; is a type of 2-oxoglutarate metabolic process [GO:0006103]; is_a GO:0006105; is a type of phosphate-containing compound metabolic process [GO:0006796]; is a type of formate metabolic process [GO:0015942]; is a type of GO:0046434; is_a monocarboxylic acid catabolic process [GO:0072329]; is part of fermentation [GO:0006113] Sources: ISBN:0716720094, MetaCyc:FERMENTATION-PWY